{
  "gene": "UniProtKB:P62502",
  "gene_symbol": "LCN6",
  "term_id": "UNKNOWN:0003",
  "gene_name": "Epididymal-specific lipocalin-6",
  "term_label": "Unknown cellular component"
}